{
  "gene": "UniProtKB:Q9H344",
  "gene_symbol": "OR51I2",
  "term_id": "UNKNOWN:0002",
  "gene_name": "Olfactory receptor 51I2",
  "term_label": "Unknown biological process"
}